{
  "term_id": "GO:0097120",
  "gene_symbol": "DLG1",
  "term_label": "receptor localization to synapse",
  "gene_name": "Disks large homolog 1",
  "gene": "UniProtKB:Q12959"
}